{
  "gene": "UniProtKB:Q8N4C7",
  "gene_name": "Syntaxin-19",
  "gene_symbol": "STX19",
  "term_label": "synaptic vesicle fusion to presynaptic active zone membrane",
  "term_id": "GO:0031629"
}